{
  "gene": "UniProtKB:O14746",
  "gene_name": "Telomerase reverse transcriptase",
  "gene_symbol": "TERT",
  "term_id": "GO:0003720",
  "term_label": "telomerase activity"
}